{
  "gene": "UniProtKB:Q13956",
  "gene_symbol": "PDE6H",
  "gene_name": "Retinal cone rhodopsin-sensitive cGMP 3',5'-cyclic phosphodiesterase subunit gamma",
  "term_id": "GO:0045742",
  "term_label": "positive regulation of epidermal growth factor receptor signaling pathway"
}